{
  "term_label": "Unknown biological process",
  "term_id": "UNKNOWN:0002",
  "gene_symbol": "C2orf49",
  "gene_name": "Ashwin",
  "gene": "UniProtKB:Q9BVC5"
}